{
  "gene_name": "T cell receptor alpha joining 25 (non-functional) (Fragment)",
  "gene": "UniProtKB:A0A075B6Z8",
  "term_label": "Unknown molecular function",
  "term_id": "UNKNOWN:0001",
  "gene_symbol": "TRAJ25"
}